{
  "gene_name": "Transmembrane protein 240",
  "term_id": "UNKNOWN:0001",
  "gene_symbol": "TMEM240",
  "term_label": "Unknown molecular function",
  "gene": "UniProtKB:Q5SV17"
}